{
  "term_id": "GO:0016740",
  "gene": "UniProtKB:E5RQL4",
  "gene_name": "Formiminotransferase N-terminal subdomain-containing protein",
  "term_label": "transferase activity",
  "gene_symbol": "FTCDNL1"
}